dendritic filopodium [GO:1902737] (cellular component) References: PMID:24464040 Sources: GOC:PARL, GOC:TermGenie, GOC:pad, GO_REF:0000064, Wikipedia:Dendritic_filopodia Note: Dendritic filopodia are generally less-well studied than dendritic spines because their transient nature makes them difficult to detect with traditional microscopy techniques, and because they are sometimes destroyed by sample preparation. Note that filopodia on dendritic shafts are distinct from other types of filopodia (even those found in dendritic growth cones) and may react differently to stimuli, as shown in PMID:12904473. Definition: A small, membranous protrusion found primarily on dendritic stretches of developing neurons. May receive synaptic input, and can develop into dendritic spines. Relationships: is a type of filopodium [GO:0030175]; is a type of neuron projection [GO:0043005]; is part of dendrite [GO:0030425] Also known as: dendrite filopodium